octamethylcyclotetrasiloxane catabolic process to dimethylsilanediol [GO:0042210] (BP) Definition: The anaerobic chemical reactions and pathways resulting in the breakdown of octamethylcyclotetrasiloxane into dimethylsilanediol. The former is a tetramer of the latter. Relationships: is a type of dimethylsilanediol metabolic process [GO:0046454]; is a type of octamethylcyclotetrasiloxane catabolic process [GO:0046517] Sources: GOC:jl Also known as: catabolic process of octamethylcyclotetrasiloxane to DMSD, catabolism of octamethylcyclotetrasiloxane to DMSD, octamethylcyclotetrasiloxane breakdown to dimethylsilanediol, octamethylcyclotetrasiloxane degradation to dimethylsilanediol